{
  "gene_name": "Methylmalonic aciduria type A protein, mitochondrial",
  "term_label": "GTPase activity",
  "gene": "UniProtKB:Q8IVH4",
  "gene_symbol": "MMAA",
  "term_id": "GO:0003924"
}